tRNA-queuosine(34) galactosyltransferase activity [GO:0141125] (molecular function) Also known as: tRNA queuosine galactosyltransferase activity, tRNA queuosine(34) galactosyltransferase activity References: PMID:37992713 Relationships: is a type of GO:0035250; is a type of catalytic activity, acting on a tRNA [GO:0140101] Definition: Catalysis of the reaction: queuosine34 in tRNA + UDP-alpha-D-galactose = H+ + O-5''-beta-D-galactosylqueuosine34 in tRNATyr + UDP. Substrates include tRNA(Tyr) and tRNA(Asp).